{
  "gene_name": "Suppressor of cytokine signaling 3",
  "gene": "UniProtKB:O14543",
  "term_label": "cytokine receptor binding",
  "gene_symbol": "SOCS3",
  "term_id": "GO:0005126"
}